{
  "gene_symbol": "CLDN15",
  "term_id": "GO:0005886",
  "term_label": "plasma membrane",
  "gene": "UniProtKB:P56746",
  "gene_name": "Claudin-15"
}